CMP catabolic process [GO:0006248] (BP) Also known as: CMP breakdown, CMP catabolism, CMP degradation Definition: The chemical reactions and pathways resulting in the breakdown of CMP, cytidine monophosphate. Relationships: is_a GO:0009175; is a type of pyrimidine ribonucleotide catabolic process [GO:0009222]; is a type of CMP metabolic process [GO:0046035] Sources: ISBN:0198506732